{
  "term_id": "UNKNOWN:0003",
  "gene_symbol": "FBXO24",
  "term_label": "Unknown cellular component",
  "gene_name": "F-box only protein 24",
  "gene": "UniProtKB:O75426"
}